{
  "gene_name": "ORM1-like protein 3",
  "gene_symbol": "ORMDL3",
  "gene": "UniProtKB:Q8N138",
  "term_label": "ceramide metabolic process",
  "term_id": "GO:0006672"
}